{
  "gene": "UniProtKB:Q6PGQ7",
  "gene_name": "Protein aurora borealis",
  "term_label": "nucleus",
  "term_id": "GO:0005634",
  "gene_symbol": "BORA"
}